{
  "term_id": "GO:0004708",
  "term_label": "MAP kinase kinase activity",
  "gene_name": "Dual specificity mitogen-activated protein kinase kinase 4",
  "gene": "UniProtKB:P45985",
  "gene_symbol": "MAP2K4"
}